{
  "term_id": "UNKNOWN:0002",
  "gene_name": "RWD domain-containing protein 2A",
  "gene_symbol": "RWDD2A",
  "gene": "UniProtKB:Q9UIY3",
  "term_label": "Unknown biological process"
}